2-deoxyglucose-6-phosphatase activity [GO:0003850] (MF) Relationships: is a type of sugar-phosphatase activity [GO:0050308] Also known as: 2-deoxy-D-glucose-6-phosphate phosphohydrolase activity, 2-deoxyglucose-6-phosphate phosphatase activity Definition: Catalysis of the reaction: 2-deoxy-D-glucose-6-phosphate + H2O = 2-deoxy-D-glucose + phosphate. Sources: EC:3.1.3.68